{
  "term_id": "GO:0007268",
  "term_label": "chemical synaptic transmission",
  "gene": "UniProtKB:Q9NZ94",
  "gene_symbol": "NLGN3",
  "gene_name": "Neuroligin-3"
}